{
  "gene_name": "Tudor domain-containing protein 3",
  "gene": "UniProtKB:Q9H7E2",
  "term_label": "histone H4 reader activity",
  "term_id": "GO:0140008",
  "gene_symbol": "TDRD3"
}